{
  "term_id": "GO:0097546",
  "gene": "UniProtKB:Q9P2H0",
  "gene_name": "Centrosomal protein of 126 kDa",
  "term_label": "ciliary base",
  "gene_symbol": "CEP126"
}